carotid body glomus cell differentiation [GO:0061103] (biological process) References: PMID:6243386 Sources: GOC:dph Relationships: is a type of GO:0061101; is part of GO:0048513 Definition: The process in which a relatively unspecialized cell acquires specialized structural and/or functional features of a glomus cell of the carotid body. The carotid body is a specialized chemosensory organ that helps respond to hypoxia.